{
  "term_id": "GO:0071144",
  "term_label": "heteromeric SMAD protein complex",
  "gene_name": "Mothers against decapentaplegic homolog 4",
  "gene": "UniProtKB:Q13485",
  "gene_symbol": "SMAD4"
}